4-methyleneglutamate-ammonia ligase activity [GO:0047581] (molecular function) Also known as: 4-methylene-L-glutamate:ammonia ligase (AMP-forming), 4-methyleneglutamine synthetase activity Definition: Catalysis of the reaction: 4-methylene-L-glutamate + ATP + NH4 = 4-methylene-L-glutamine + AMP + diphosphate + 2 H+. Sources: EC:6.3.1.7, RHEA:13853 Relationships: is a type of GO:0016880